{
  "gene": "UniProtKB:Q6ZS52",
  "gene_name": "Putative uncharacterized protein FLJ45825",
  "gene_symbol": "Q6ZS52",
  "term_id": "UNKNOWN:0003",
  "term_label": "Unknown cellular component"
}